chromosomal 5-methylcytosine DNA demethylation pathway [GO:0141166] (biological process) Definition: A process that chemically modifies 5-methylcytosine (5meC) to make it a substrate for the base excision repair pathway, which then restores the unmodified cytosine. Also known as: epigenetic 5-methylcytosine DNA demethylation, epigenetic 5-methylcytosine DNA demethylation pathway, epigenetic DNA demethylation Subtypes: chromosomal 5-methylcytosine DNA demethylation, oxidation pathway [GO:0141167], chromosomal 5-methylcytosine DNA demethylation, oxidative deamination pathway [GO:0141168], chromosomal 5-methylcytosine DNA demethylation, direct 5-methylcytosine excision pathway [GO:0141169] Note: Note that this term describes the biochemical pathways of chromosomal cytosine demethylation but is agnostic to the effect on gene expression. If the data supports it, consider co-annotating to 'positive regulation of gene expression, epigenetic ; GO:0044029' or a child. References: PMID:21862972, PMID:31546611, PMID:36478523 Relationships: is a type of DNA metabolic process [GO:0006259]